{
  "gene": "UniProtKB:Q13601",
  "term_label": "Unknown molecular function",
  "gene_name": "KRR1 small subunit processome component homolog",
  "gene_symbol": "KRR1",
  "term_id": "UNKNOWN:0001"
}